{
  "gene_name": "Dihydropyrimidine dehydrogenase [NADP(+)]",
  "term_id": "GO:0006210",
  "gene_symbol": "DPYD",
  "gene": "UniProtKB:Q12882",
  "term_label": "thymine catabolic process"
}